{
  "term_label": "protein serine/threonine phosphatase activity",
  "term_id": "GO:0004722",
  "gene": "UniProtKB:Q8WVY7",
  "gene_name": "Ubiquitin-like domain-containing CTD phosphatase 1",
  "gene_symbol": "UBLCP1"
}